{
  "gene_name": "ATP-dependent RNA helicase DDX39A",
  "gene_symbol": "DDX39A",
  "term_label": "mRNA export from nucleus",
  "term_id": "GO:0006406",
  "gene": "UniProtKB:O00148"
}